{
  "gene_symbol": "CNGA2",
  "term_label": "sensory perception of chemical stimulus",
  "gene": "UniProtKB:Q16280",
  "term_id": "GO:0007606",
  "gene_name": "Cyclic nucleotide-gated olfactory channel"
}